positive regulation of secondary cell wall biogenesis [GO:1901348] (biological process) Sources: GOC:TermGenie Relationships: is_a GO:0044089; is a type of GO:1903340; is a type of GO:2000652; positively regulates plant-type secondary cell wall biogenesis [GO:0009834] Also known as: activation of secondary cell wall anabolism, activation of secondary cell wall biosynthetic process, activation of secondary cell wall formation, activation of secondary cell wall synthesis, positive regulation of secondary cell wall anabolism, positive regulation of secondary cell wall biosynthetic process, positive regulation of secondary cell wall formation, positive regulation of secondary cell wall synthesis, up regulation of secondary cell wall anabolism, up regulation of secondary cell wall biosynthetic process, up regulation of secondary cell wall formation, up regulation of secondary cell wall synthesis, up-regulation of secondary cell wall anabolism, up-regulation of secondary cell wall biosynthetic process, up-regulation of secondary cell wall formation, up-regulation of secondary cell wall synthesis, upregulation of secondary cell wall anabolism, upregulation of secondary cell wall biosynthetic process, upregulation of secondary cell wall formation, upregulation of secondary cell wall synthesis, activation of cellulose and pectin-containing secondary cell wall biogenesis, activation of plant-type secondary cell wall biogenesis, positive regulation of cellulose and pectin-containing secondary cell wall biogenesis, positive regulation of plant-type secondary cell wall biogenesis, up regulation of cellulose and pectin-containing secondary cell wall biogenesis, up regulation of plant-type secondary cell wall biogenesis, up regulation of secondary cell wall biogenesis, up-regulation of cellulose and pectin-containing secondary cell wall biogenesis, up-regulation of plant-type secondary cell wall biogenesis, up-regulation of secondary cell wall biogenesis, upregulation of cellulose and pectin-containing secondary cell wall biogenesis, upregulation of plant-type secondary cell wall biogenesis, upregulation of secondary cell wall biogenesis, activation of secondary cell wall biogenesis Definition: Any process that activates or increases the frequency, rate or extent of secondary cell wall biogenesis.